{
  "term_id": "GO:2000134",
  "term_label": "negative regulation of G1/S transition of mitotic cell cycle",
  "gene": "UniProtKB:Q63ZY3",
  "gene_name": "KN motif and ankyrin repeat domain-containing protein 2",
  "gene_symbol": "KANK2"
}